{
  "gene_symbol": "PRKCG",
  "gene_name": "Protein kinase C gamma type",
  "term_id": "GO:0004674",
  "term_label": "protein serine/threonine kinase activity",
  "gene": "UniProtKB:P05129"
}